{
  "gene_symbol": "OASL",
  "term_label": "negative regulation of viral genome replication",
  "gene_name": "2'-5'-oligoadenylate synthase-like protein",
  "gene": "UniProtKB:Q15646",
  "term_id": "GO:0045071"
}